{
  "gene_symbol": "RAX2",
  "gene": "UniProtKB:Q96IS3",
  "gene_name": "Retina and anterior neural fold homeobox protein 2",
  "term_id": "UNKNOWN:0003",
  "term_label": "Unknown cellular component"
}